ether lipid metabolic process [GO:0046485] (biological process) Relationships: is a type of lipid metabolic process [GO:0006629] Subtypes: ether lipid biosynthetic process [GO:0008611], platelet activating factor metabolic process [GO:0046469] Definition: The chemical reactions and pathways involving ether lipids, lipids that contain (normally) one lipid alcohol in ether linkage to one of the carbon atoms (normally C-1) of glycerol. References: PMID:15337120 Sources: ISBN:0198506732 Also known as: ether lipid metabolism, plasmalogen metabolic process